{
  "gene_name": "Centrosomal protein of 76 kDa",
  "gene": "UniProtKB:Q8TAP6",
  "term_id": "UNKNOWN:0001",
  "term_label": "Unknown molecular function",
  "gene_symbol": "CEP76"
}